receptor decoy activity [GO:0140319] (molecular function) Also known as: decoy receptor, decoy death receptor activity Definition: Binding and sequestering a specific receptor ligand to prevent it from binding to its regular receptor. Subtypes: GO:0140320 Relationships: is a type of molecular sequestering activity [GO:0140313] Sources: Wikipedia:Decoy_receptors